{
  "gene": "UniProtKB:Q9NV79",
  "gene_name": "Protein-L-isoaspartate O-methyltransferase domain-containing protein 2",
  "gene_symbol": "PCMTD2",
  "term_label": "protein-L-isoaspartate (D-aspartate) O-methyltransferase activity",
  "term_id": "GO:0004719"
}